synaptic signaling [GO:0099536] (biological process) Definition: Cell-cell signaling to, from or within a synapse. Relationships: is a type of GO:0007267; occurs in synapse [GO:0045202] Subtypes: synaptic signaling by nitric oxide [GO:0099163], trans-synaptic signaling [GO:0099537], synaptic signaling via neuropeptide [GO:0099538] Sources: GOC:dos